purine nucleoside bisphosphate metabolic process [GO:0034032] (biological process) Relationships: is a type of nucleoside bisphosphate metabolic process [GO:0033865]; is a type of GO:0072521 Subtypes: purine nucleoside bisphosphate biosynthetic process [GO:0034033], GO:0034034, purine ribonucleoside bisphosphate metabolic process [GO:0034035] Definition: The chemical reactions and pathways involving a purine nucleoside bisphosphate, a compound consisting of a purine base linked to a deoxyribose or ribose sugar esterified with one phosphate group attached to each of two different hydroxyl groups on the sugar. Also known as: purine nucleoside bisphosphate metabolism Sources: GOC:mah, GOC:pde